{
  "term_label": "Unknown molecular function",
  "term_id": "UNKNOWN:0001",
  "gene_name": "Putative uncharacterized protein HSD52",
  "gene": "UniProtKB:Q0P140",
  "gene_symbol": "HSD52"
}